{
  "gene": "UniProtKB:Q71UM5",
  "term_label": "cytosolic small ribosomal subunit",
  "gene_name": "Ribosomal protein eS27-like",
  "term_id": "GO:0022627",
  "gene_symbol": "RPS27L"
}